{
  "term_id": "GO:0005634",
  "term_label": "nucleus",
  "gene_symbol": "BUB1",
  "gene": "UniProtKB:O43683",
  "gene_name": "Mitotic checkpoint serine_threonine-protein kinase BUB1"
}